{
  "gene_symbol": "SEMA3F",
  "gene_name": "Semaphorin-3F",
  "term_id": "GO:0007411",
  "term_label": "axon guidance",
  "gene": "UniProtKB:Q13275"
}